{
  "gene": "UniProtKB:Q9BQY4",
  "gene_symbol": "RHOXF2",
  "gene_name": "Rhox homeobox family member 2",
  "term_label": "regulation of transcription by RNA polymerase II",
  "term_id": "GO:0006357"
}